{
  "gene_name": "Proprotein convertase subtilisin_kexin type 6",
  "gene": "UniProtKB:P29122",
  "term_id": "GO:0005615",
  "gene_symbol": "PCSK6",
  "term_label": "extracellular space"
}